{
  "term_id": "UNKNOWN:0002",
  "term_label": "Unknown biological process",
  "gene_name": "N-alpha-acetyltransferase 11",
  "gene": "UniProtKB:Q9BSU3",
  "gene_symbol": "NAA11"
}